orthodenticle mRNA localization [GO:0060812] (biological process) Also known as: orthodenticle mRNA localisation Relationships: is a type of intracellular mRNA localization involved in anterior/posterior axis specification [GO:0060811] Sources: GOC:dph, GOC:sdb_2009, GOC:tb Definition: Any process in which orthodenticle mRNA is transported to and maintained in the oocyte and/or syncytial embryo as part of the process that will specify the anterior/posterior axis.